{
  "gene": "UniProtKB:P63104",
  "term_id": "GO:0008104",
  "gene_symbol": "YWHAZ",
  "term_label": "intracellular protein localization",
  "gene_name": "14-3-3 protein zeta_delta"
}